malate transmembrane transport [GO:0071423] (biological process) Also known as: malate membrane transport, transmembrane malate transport Note: Note that this term is not intended for use in annotating lateral movement within membranes. Sources: GOC:mah Subtypes: malate import across plasma membrane [GO:0098714] Relationships: is a type of GO:0015743; is a type of carboxylic acid transmembrane transport [GO:1905039] Definition: A process in which a malate ion is transported across a membrane.